bombesin receptor binding [GO:0031705] (molecular function) Relationships: is a type of neuropeptide receptor binding [GO:0071855] Also known as: bombesin receptor ligand Subtypes: GO:0031706, endothelin A receptor binding [GO:0031707], endothelin B receptor binding [GO:0031708], GO:0031709, GO:0031710 Definition: Binding to a bombesin receptor. Sources: GOC:mah, GOC:nln